{
  "gene_symbol": "NCF1",
  "gene": "UniProtKB:P14598",
  "gene_name": "Neutrophil cytosol factor 1",
  "term_label": "superoxide anion generation",
  "term_id": "GO:0042554"
}